{
  "gene_name": "DnaJ homolog subfamily B member 14",
  "gene": "UniProtKB:Q8TBM8",
  "gene_symbol": "DNAJB14",
  "term_id": "GO:0006457",
  "term_label": "protein folding"
}